{
  "gene_symbol": "CDX4",
  "term_label": "DNA-binding transcription factor activity",
  "gene_name": "Homeobox protein CDX-4",
  "gene": "UniProtKB:O14627",
  "term_id": "GO:0003700"
}